{
  "term_id": "GO:1990841",
  "gene_symbol": "ZNF750",
  "term_label": "promoter-specific chromatin binding",
  "gene_name": "Zinc finger protein 750",
  "gene": "UniProtKB:Q32MQ0"
}